lipoprotein localization to outer membrane [GO:0044874] (biological process) Relationships: is a type of lipoprotein localization to membrane [GO:0044873] Sources: GOC:jl Definition: A process in which a lipoprotein is transported to, or maintained in, a specific location in an outer membrane.